{
  "term_label": "regulation of DNA-templated transcription",
  "gene_symbol": "KDM5A",
  "gene": "UniProtKB:P29375",
  "term_id": "GO:0006355",
  "gene_name": "Lysine-specific demethylase 5A"
}